mesenchymal stem cell proliferation [GO:0097168] (biological process) Subtypes: mesenchymal stem cell proliferation involved in nephron morphogenesis [GO:0072090] References: PMID:20626275 Sources: CL:0000134, GOC:yaf Also known as: MSC proliferation Definition: The multiplication or reproduction of mesenchymal stem cells, resulting in the expansion of a stem cell population. A mesenchymal stem cell, or MSC, is a cell that retains the ability to divide and proliferate throughout life to provide progenitor cells that can differentiate into specialized mesenchymal cells. Regulation: regulated by regulation of mesenchymal stem cell proliferation [GO:1902460]; negatively regulated by negative regulation of mesenchymal stem cell proliferation [GO:1902461]; positively regulated by positive regulation of mesenchymal stem cell proliferation [GO:1902462] Relationships: is a type of stem cell proliferation [GO:0072089]